{
  "gene_symbol": "TOLLIP",
  "gene_name": "Toll-interacting protein",
  "gene": "UniProtKB:Q9H0E2",
  "term_label": "ubiquitin conjugating enzyme binding",
  "term_id": "GO:0031624"
}